{
  "term_id": "GO:0005852",
  "term_label": "eukaryotic translation initiation factor 3 complex",
  "gene_name": "Eukaryotic translation initiation factor 3 subunit J",
  "gene": "UniProtKB:O75822",
  "gene_symbol": "EIF3J"
}